splicing factor binding [GO:1990935] (molecular function) Definition: Binding to a protein involved in the process of removing sections of the primary RNA transcript to form the mature form of the RNA. References: PMID:11118435 Relationships: is a type of protein binding [GO:0005515]